{
  "gene_name": "Sialic acid-binding Ig-like lectin 8",
  "gene": "UniProtKB:Q9NYZ4",
  "term_id": "GO:0033691",
  "gene_symbol": "SIGLEC8",
  "term_label": "sialic acid binding"
}